all-trans-nonaprenyl-diphosphate synthase (geranylgeranyl-diphosphate specific) activity [GO:0052924] (molecular function) Definition: Catalysis of the reaction: 5 isopentenyl diphosphate + (2E,6E,10E)-geranylgeranyl diphosphate = all-trans-nonaprenyl diphosphate + 5 diphosphate. Sources: RHEA:27594 Relationships: is a type of GO:0120531 Also known as: nonaprenyl diphosphate synthase activity, solanesyl diphosphate synthase activity, solanesyl diphosphate synthetase activity